glutamate-gated receptor activity [GO:0004970] (molecular function) Note: Note that this term represents an activity and not a gene product. Consider also annotating to the molecular function terms 'glutamate-gated ion channel activity ; GO:0005234' and 'cation channel activity ; GO:0005261'. Relationships: is a type of glutamate receptor activity [GO:0008066]; is a type of amino acid transmembrane transporter activity [GO:0015171]; is a type of GO:0022824; is a type of carboxylic acid transmembrane transporter activity [GO:0046943]; is part of ionotropic glutamate receptor signaling pathway [GO:0035235] Sources: ISBN:0198506732 Subtypes: AMPA glutamate receptor activity [GO:0004971], NMDA glutamate receptor activity [GO:0004972], kainate selective glutamate receptor activity [GO:0015277], glutamate-gated calcium ion channel activity [GO:0022849] Also known as: ionotropic glutamate receptor activity Definition: Catalysis of the transmembrane transfer of an ion by a channel that opens when glutamate has been bound by the channel complex or one of its constituent parts.